{
  "gene": "UniProtKB:A0A1B0GVS7",
  "term_label": "nucleus",
  "gene_name": "MyoD family inhibitor domain-containing protein 2",
  "term_id": "GO:0005634",
  "gene_symbol": "MDFIC2"
}